{
  "term_label": "regulation of potassium ion transmembrane transport",
  "gene_symbol": "KCNIP3",
  "term_id": "GO:1901379",
  "gene": "UniProtKB:Q9Y2W7",
  "gene_name": "Calsenilin"
}